dipeptide transmembrane transporter activity [GO:0071916] (molecular function) Also known as: dipeptide transporter activity Subtypes: secondary active p-aminobenzoyl-glutamate transmembrane transporter activity [GO:0015558], GO:0042933, dipeptide uniporter activity [GO:0160178] Definition: Enables the transfer of a dipeptide from one side of a membrane to the other. A dipeptide is a combination of two amino acids linked together by a peptide (-CO-NH-) bond. Sources: GOC:mah Relationships: is a type of oligopeptide transmembrane transporter activity [GO:0035673]; is part of dipeptide transmembrane transport [GO:0035442]